{
  "term_label": "plasma membrane",
  "gene_symbol": "TRBV6-6",
  "gene_name": "T cell receptor beta variable 6-6",
  "term_id": "GO:0005886",
  "gene": "UniProtKB:A0A0A6YYG2"
}